{
  "gene": "UniProtKB:Q86SZ2",
  "gene_symbol": "TRAPPC6B",
  "gene_name": "Trafficking protein particle complex subunit 6B",
  "term_id": "GO:0030008",
  "term_label": "TRAPP complex"
}